{
  "term_label": "regulation of G protein-coupled receptor signaling pathway",
  "gene_name": "Regulator of G-protein signaling 14",
  "gene_symbol": "RGS14",
  "gene": "UniProtKB:O43566",
  "term_id": "GO:0008277"
}